{
  "term_label": "nucleosome array spacer activity",
  "gene": "UniProtKB:O60264",
  "term_id": "GO:0140750",
  "gene_symbol": "SMARCA5",
  "gene_name": "SWI_SNF-related matrix-associated actin-dependent regulator of chromatin subfamily A member 5"
}